{
  "term_id": "GO:0000791",
  "gene_name": "Histone H1.5",
  "gene": "UniProtKB:P16401",
  "gene_symbol": "H1-5",
  "term_label": "euchromatin"
}